{
  "term_label": "NSL complex",
  "term_id": "GO:0044545",
  "gene": "UniProtKB:A8MW92",
  "gene_name": "PHD finger protein 20-like protein 1",
  "gene_symbol": "PHF20L1"
}